{
  "term_id": "GO:0006888",
  "gene_name": "Coatomer subunit gamma-2",
  "gene": "UniProtKB:Q9UBF2",
  "gene_symbol": "COPG2",
  "term_label": "endoplasmic reticulum to Golgi vesicle-mediated transport"
}